{
  "term_label": "plasma membrane",
  "term_id": "GO:0005886",
  "gene_name": "Olfactory receptor 2T11",
  "gene_symbol": "OR2T11",
  "gene": "UniProtKB:Q8NH01"
}